{
  "term_id": "GO:0005634",
  "term_label": "nucleus",
  "gene": "UniProtKB:Q9H2Z4",
  "gene_name": "Homeobox protein Nkx-2.4",
  "gene_symbol": "NKX2-4"
}